acetyl-CoA biosynthetic process [GO:0006085] (biological process) Sources: GOC:go_curators Also known as: acetyl-CoA anabolism, acetyl-CoA biosynthesis, acetyl-CoA formation, acetyl-CoA synthesis Relationships: is a type of acetyl-CoA metabolic process [GO:0006084]; is a type of acyl-CoA biosynthetic process [GO:0071616] Subtypes: pyruvate decarboxylation to acetyl-CoA [GO:0006086], acetyl-CoA biosynthetic process from acetate [GO:0019427], acetyl-CoA biosynthetic process from ethanol [GO:0019431], GO:0030634, acetyl-CoA biosynthetic process from pantothenate [GO:1990181] Definition: The chemical reactions and pathways resulting in the formation of acetyl-CoA, a derivative of coenzyme A in which the sulfhydryl group is acetylated.